{
  "gene_name": "Breast cancer type 2 susceptibility protein",
  "term_label": "double-strand break repair via homologous recombination",
  "gene_symbol": "BRCA2",
  "term_id": "GO:0000724",
  "gene": "UniProtKB:P51587"
}